{
  "gene_symbol": "WASHC2A",
  "gene": "UniProtKB:Q641Q2",
  "term_label": "protein localization to endosome",
  "term_id": "GO:0036010",
  "gene_name": "WASH complex subunit 2A"
}